negative regulation of interleukin-17 production [GO:0032700] (BP) Relationships: is a type of negative regulation of cytokine production [GO:0001818]; is a type of GO:0032660; negatively regulates interleukin-17 production [GO:0032620] Definition: Any process that stops, prevents, or reduces the frequency, rate, or extent of production of any member of the interleukin-17 family of cytokines. Subtypes: negative regulation of interleukin-17A production [GO:0150152] References: PMID:16482511 Sources: GOC:add, GOC:mah Also known as: down regulation of interleukin-17 production, downregulation of interleukin-17 production, negative regulation of Cytotoxic T-lymphocyte-associated antigen 8 secretion, negative regulation of IL-17 production, inhibition of interleukin-17 production, negative regulation of CTLA-8 production, negative regulation of interleukin-17 biosynthetic process, negative regulation of interleukin-17 secretion